{
  "gene": "UniProtKB:P43115",
  "gene_symbol": "PTGER3",
  "term_label": "phospholipase C-activating G protein-coupled receptor signaling pathway",
  "gene_name": "Prostaglandin E2 receptor EP3 subtype",
  "term_id": "GO:0007200"
}